diglucosyl diacylglycerol synthase activity [GO:0047257] (MF) Sources: EC:2.4.1.208, MetaCyc:2.4.1.208-RXN Also known as: diglucosyl diacylglycerol (DGlcDAG) synthase activity, DGlcDAG synthase activity, MGlcDAG (1->2) glucosyltransferase activity, UDP-glucose:1,2-diacyl-3-O-(alpha-D-glucopyranosyl)-sn-glycerol (1->2) glucosyltransferase activity, monoglucosyl diacylglycerol (1->2) glucosyltransferase activity Relationships: is a type of UDP-glycosyltransferase activity [GO:0008194]; is a type of hexosyltransferase activity [GO:0016758] Definition: Catalysis of the reaction: 1,2-diacyl-3-O-(alpha-D-glucopyranosyl)-sn-glycerol + UDP-D-glucose = UDP + 1,2-diacyl-3-O-(alpha-D-glucopyranosyl(1,2)-O-alpha-D-glucopyranosyl)-sn-glycerol.